{
  "gene_name": "Toll-like receptor 8",
  "term_id": "GO:0002224",
  "gene_symbol": "TLR8",
  "gene": "UniProtKB:Q9NR97",
  "term_label": "toll-like receptor signaling pathway"
}